binding of sperm to zona pellucida [GO:0007339] (BP) Also known as: ZPG binding Relationships: is a type of sperm-egg recognition [GO:0035036] Sources: GOC:dph, ISBN:0878932437 Definition: The process in which the sperm binds to the zona pellucida glycoprotein layer of the egg. The process begins with the attachment of the sperm plasma membrane to the zona pellucida and includes attachment of the acrosome inner membrane to the zona pellucida after the acrosomal reaction takes place. Regulation: regulated by regulation of binding of sperm to zona pellucida [GO:2000359]; negatively regulated by negative regulation of binding of sperm to zona pellucida [GO:2000360]